{
  "term_id": "GO:0035494",
  "gene_symbol": "NAPA",
  "term_label": "SNARE complex disassembly",
  "gene_name": "Alpha-soluble NSF attachment protein",
  "gene": "UniProtKB:P54920"
}